{
  "term_label": "ubiquitin-dependent protein catabolic process",
  "term_id": "GO:0006511",
  "gene_name": "Roquin-1",
  "gene": "UniProtKB:Q5TC82",
  "gene_symbol": "RC3H1"
}